{
  "gene_name": "Leukosialin",
  "term_id": "GO:0042742",
  "gene_symbol": "SPN",
  "gene": "UniProtKB:P16150",
  "term_label": "defense response to bacterium"
}